{
  "gene": "UniProtKB:P08861",
  "term_label": "proteolysis",
  "gene_name": "Chymotrypsin-like elastase family member 3B",
  "gene_symbol": "CELA3B",
  "term_id": "GO:0006508"
}